{
  "gene_symbol": "NTAQ1",
  "term_label": "cytosol",
  "term_id": "GO:0005829",
  "gene": "UniProtKB:Q96HA8",
  "gene_name": "Protein N-terminal glutamine amidohydrolase"
}